{
  "gene_symbol": "BRWD1",
  "term_id": "GO:0006357",
  "term_label": "regulation of transcription by RNA polymerase II",
  "gene": "UniProtKB:Q9NSI6",
  "gene_name": "Bromodomain and WD repeat-containing protein 1"
}